{
  "term_label": "estrogen receptor signaling pathway",
  "gene_name": "Estrogen receptor beta",
  "gene_symbol": "ESR2",
  "term_id": "GO:0030520",
  "gene": "UniProtKB:Q92731"
}